{
  "term_label": "ATPase inhibitor activity",
  "term_id": "GO:0042030",
  "gene_name": "Cardiac phospholamban",
  "gene": "UniProtKB:P26678",
  "gene_symbol": "PLN"
}